{
  "term_label": "regulation of gene expression",
  "gene_symbol": "PRDM6",
  "term_id": "GO:0010468",
  "gene_name": "Putative histone-lysine N-methyltransferase PRDM6",
  "gene": "UniProtKB:Q9NQX0"
}